{
  "term_id": "GO:0006302",
  "gene_symbol": "UIMC1",
  "gene": "UniProtKB:Q96RL1",
  "gene_name": "BRCA1-A complex subunit RAP80",
  "term_label": "double-strand break repair"
}